2-oxoaldehyde dehydrogenase (NAD+) activity [GO:0047551] (molecular function) Sources: EC:1.2.1.23, MetaCyc:2-OXOALDEHYDE-DEHYDROGENASE-NAD+-RXN Definition: Catalysis of the reaction: a 2-oxoaldehyde + NAD+ + H2O = a 2-oxo acid + NADH + H+. Relationships: is a type of aldehyde dehydrogenase (NAD+) activity [GO:0004029] Also known as: 2-ketoaldehyde dehydrogenase, alpha-ketoaldehyde dehydrogenase activity, methylglyoxal dehydrogenase activity, 2-oxoaldehyde dehydrogenase (NAD+), 2-oxoaldehyde:NAD+ 2-oxidoreductase activity, NAD-dependent alpha-ketoaldehyde dehydrogenase activity, NAD-linked alpha-ketoaldehyde dehydrogenase activity